nucleoside phosphate biosynthetic process [GO:1901293] (biological process) Definition: The chemical reactions and pathways resulting in the formation of a nucleoside phosphate. Sources: GOC:TermGenie Also known as: nucleoside phosphate anabolism, nucleoside phosphate biosynthesis, nucleoside phosphate formation, nucleoside phosphate synthesis Relationships: is a type of nucleoside phosphate metabolic process [GO:0006753]; is a type of nucleobase-containing compound biosynthetic process [GO:0034654]; is a type of GO:0090407 Subtypes: GO:0009124, nucleoside diphosphate biosynthetic process [GO:0009133], nucleoside triphosphate biosynthetic process [GO:0009142], nucleotide biosynthetic process [GO:0009165], GO:0009226, GO:0015937, GDP-alpha-D-mannosylchitobiosyldiphosphodolichol biosynthetic process [GO:0019347], nucleoside bisphosphate biosynthetic process [GO:0033866], acyl-CoA biosynthetic process [GO:0071616]